{
  "gene_symbol": "ZNF239",
  "term_id": "GO:0006357",
  "term_label": "regulation of transcription by RNA polymerase II",
  "gene": "UniProtKB:Q16600",
  "gene_name": "Zinc finger protein 239"
}